{
  "gene_symbol": "FTSJ3",
  "term_id": "GO:0005730",
  "gene_name": "pre-rRNA 2'-O-ribose RNA methyltransferase FTSJ3",
  "term_label": "nucleolus",
  "gene": "UniProtKB:Q8IY81"
}